{
  "gene_name": "Immunoglobulin kappa variable 1-8",
  "term_label": "Unknown molecular function",
  "gene": "UniProtKB:A0A0C4DH67",
  "gene_symbol": "IGKV1-8",
  "term_id": "UNKNOWN:0001"
}